growth plate cartilage chondrocyte division [GO:0003423] (biological process) Definition: The process resulting in the oriented physical partitioning and separation of a chondrocytes in the growth plate. Sources: GOC:ascb_2009, GOC:dph, GOC:tb Relationships: is a type of cell division [GO:0051301]; BFO_0000050 growth plate cartilage chondrocyte proliferation [GO:0003419]